plasma membrane-derived thylakoid lumen [GO:0031979] (CC) Sources: GOC:mah, GOC:mtg_sensu Definition: The volume enclosed by a plasma membrane-derived thylakoid. Relationships: is a type of GO:0031977; is a type of GO:0060205; is part of GO:0005886; BFO_0000050 bacterial thylakoid [GO:0030075] Also known as: plasma membrane thylakoid lumen